urea cycle [GO:0000050] (biological process) Sources: GOC:pde, GOC:vw, ISBN:0198506732 Also known as: ornithine cycle, urea biosynthesis, urea biosynthetic process Definition: The sequence of reactions by which arginine is synthesized from ornithine, then cleaved to yield urea and regenerate ornithine. The overall reaction equation is NH3 + CO2 + aspartate + 3 ATP + 2 H2O = urea + fumarate + 2 ADP + 2 phosphate + AMP + diphosphate. Relationships: is a type of GO:0019627; is a type of GO:0043604